{
  "gene_symbol": "DIDO1",
  "term_id": "UNKNOWN:0002",
  "gene": "UniProtKB:Q9BTC0",
  "term_label": "Unknown biological process",
  "gene_name": "Death-inducer obliterator 1"
}